regulation of mitotic DNA replication initiation from late origin [GO:0101017] (biological process) Definition: Any process that modulates the frequency, rate or extent of firing from a late origin of replication involved in mitotic DNA replication. Subtypes: GO:0101018 Relationships: is a type of regulation of mitotic DNA replication initiation [GO:1903466] References: PMID:26436827 Also known as: regulation of late replication origin firing